lymphocyte homeostasis [GO:0002260] (biological process) Definition: The process of regulating the proliferation and elimination of lymphocytes such that the total number of lymphocytes within a whole or part of an organism is stable over time in the absence of an outside stimulus. References: PMID:15826826, PMID:16319493, PMID:16551252, PMID:16551262 Sources: GOC:add Subtypes: B cell homeostasis [GO:0001782], mucosal lymphocyte homeostasis [GO:0002261], T cell homeostasis [GO:0043029] Relationships: is a type of leukocyte homeostasis [GO:0001776]